{
  "gene": "UniProtKB:B5MCN3",
  "gene_symbol": "SEC14L6",
  "gene_name": "Putative SEC14-like protein 6",
  "term_label": "Unknown molecular function",
  "term_id": "UNKNOWN:0001"
}